{
  "gene_name": "Sex comb on midleg-like protein 2",
  "gene_symbol": "SCML2",
  "gene": "UniProtKB:Q9UQR0",
  "term_label": "chromatin binding",
  "term_id": "GO:0003682"
}